{
  "gene": "UniProtKB:Q13224",
  "term_id": "GO:0017146",
  "term_label": "NMDA selective glutamate receptor complex",
  "gene_name": "Glutamate receptor ionotropic, NMDA 2B",
  "gene_symbol": "GRIN2B"
}